microfibril binding [GO:0050436] (molecular function) Note: See also the cellular component term 'microfibril ; GO:0001527'. Relationships: is a type of extracellular matrix binding [GO:0050840] Sources: GOC:ai Definition: Binding to a microfibril, any small fibril occurring in biological material.